positive regulation of establishment of blood-brain barrier [GO:0090211] (BP) Also known as: positive regulation of establishment of BBB Relationships: is a type of positive regulation of cell development [GO:0010720]; is a type of GO:0090210; positively regulates establishment of blood-brain barrier [GO:0060856] Sources: GOC:BHF, GOC:dph, GOC:tb Definition: Any process that increases the rate, frequency or extent of the establishment of the blood-brain barrier, a selectively permeable structural and functional barrier that exists between the capillaries and the brain.